{
  "gene_name": "Lipocalin-15",
  "term_id": "UNKNOWN:0002",
  "gene": "UniProtKB:Q6UWW0",
  "term_label": "Unknown biological process",
  "gene_symbol": "LCN15"
}